kinin cascade [GO:0002254] (biological process) Relationships: is a type of GO:0002526; is a type of protein activation cascade [GO:0072376] Definition: A series of reactions that takes place outside the cell that occur as a result of by-products of tissue damage, including collagen, cartilage, and basement membrane. The ultimate product of the kinin cascade include kallidin and bradykinin, agents known to induce smooth muscle contraction, vasoconstriction, and increased vascular permeability. Regulation: RO_0002211 by GO:0002256; negatively regulated by GO:0002257; positively regulated by positive regulation of kinin cascade [GO:0002258] Subtypes: tissue kallikrein-kinin cascade [GO:0002255], plasma kallikrein-kinin cascade [GO:0002353] References: PMID:11842287, PMID:14501145 Sources: GOC:jal, ISBN:0721601871